{
  "gene_symbol": "FADS3",
  "gene": "UniProtKB:Q9Y5Q0",
  "term_label": "oxidoreductase activity, acting on paired donors, with oxidation of a pair of donors resulting in the reduction of molecular oxygen to two molecules of water",
  "term_id": "GO:0016717",
  "gene_name": "Fatty acid desaturase 3"
}